{
  "term_id": "GO:0015630",
  "gene_symbol": "SEPTIN7",
  "gene": "UniProtKB:Q16181",
  "term_label": "microtubule cytoskeleton",
  "gene_name": "Septin-7"
}